{
  "term_id": "GO:0070098",
  "gene": "UniProtKB:P48061",
  "term_label": "chemokine-mediated signaling pathway",
  "gene_symbol": "CXCL12",
  "gene_name": "Stromal cell-derived factor 1"
}